{
  "gene": "UniProtKB:P12872",
  "gene_symbol": "MLN",
  "gene_name": "Promotilin",
  "term_id": "UNKNOWN:0003",
  "term_label": "Unknown cellular component"
}